symbiont-mediated perturbation of host exit from mitosis [GO:0039593] (biological process) Also known as: inhibition of host mitotic exit by virus, perturbation by virus of host exit from mitosis, suppression by virus of host exit from mitosis Definition: A process in which a virus interferes with the host cell completing the M phase of the cell cycle. Sources: VZ:877 Relationships: is a type of symbiont-mediated perturbation of host cell cycle progression [GO:0044071]